{
  "term_id": "GO:0036157",
  "gene_name": "Dynein axonemal intermediate chain 2",
  "gene_symbol": "DNAI2",
  "term_label": "outer dynein arm",
  "gene": "UniProtKB:Q9GZS0"
}